{
  "term_label": "Unknown biological process",
  "term_id": "UNKNOWN:0002",
  "gene_name": "Putative uncharacterized protein PRO2289",
  "gene": "UniProtKB:Q9P1D8",
  "gene_symbol": "PRO2289"
}